{
  "gene_symbol": "CFL2",
  "term_id": "GO:0030043",
  "gene": "UniProtKB:Q9Y281",
  "term_label": "actin filament fragmentation",
  "gene_name": "Cofilin-2"
}